{
  "gene_symbol": "L2HGDH",
  "term_label": "mitochondrion",
  "gene": "UniProtKB:Q9H9P8",
  "term_id": "GO:0005739",
  "gene_name": "L-2-hydroxyglutarate dehydrogenase, mitochondrial"
}